{
  "gene_symbol": "EVA1C",
  "term_id": "GO:0005576",
  "term_label": "extracellular region",
  "gene_name": "Protein eva-1 homolog C",
  "gene": "UniProtKB:P58658"
}